{
  "term_label": "guanyl-nucleotide exchange factor activity",
  "gene_name": "DENN domain-containing protein 4B",
  "term_id": "GO:0005085",
  "gene_symbol": "DENND4B",
  "gene": "UniProtKB:O75064"
}